negative regulation of high-density lipoprotein particle clearance [GO:0010987] (biological process) Definition: Any process that decreases the rate, frequency or extent of high-density lipoprotein particle clearance. High-density lipoprotein particle clearance is the process in which a high-density lipoprotein particle is removed from the blood via receptor-mediated endocytosis and its constituent parts degraded. Relationships: is a type of regulation of high-density lipoprotein particle clearance [GO:0010982]; is a type of GO:0010985; negatively regulates GO:0034384 Sources: GOC:BHF, GOC:dph, GOC:tb